cellular response to chemical stimulus [GO:0070887] (biological process) Note: Note that this term is in the subset of terms that should not be used for direct gene product annotation. Instead, select a child term or, if no appropriate child term exists, please request a new term. Direct annotations to this term may be amended during annotation QC. Sources: GOC:mah Relationships: is a type of response to chemical [GO:0042221]; is a type of cellular response to stimulus [GO:0051716] Definition: Any process that results in a change in state or activity of a cell (in terms of movement, secretion, enzyme production, gene expression, etc.) as a result of a chemical stimulus. Subtypes: cellular response to nutrient [GO:0031670], cellular response to hormone stimulus [GO:0032870], cellular response to chemical stress [GO:0062197], GO:0071229, cellular response to antibiotic [GO:0071236], cellular response to food [GO:0071240], cellular response to arsenic-containing substance [GO:0071243], cellular response to metal ion [GO:0071248], cellular response to nicotine [GO:0071316], cellular response to lipid [GO:0071396], cellular response to cycloalkane [GO:0071408], cellular response to fluoxetine [GO:0071411], cellular response to pheromone [GO:0071444], GO:0071453, cellular response to xenobiotic stimulus [GO:0071466], cellular response to epinephrine stimulus [GO:0071872], cellular response to bismuth [GO:0072701], cellular response to cisplatin [GO:0072719], cellular response to Gentian violet [GO:0072729], GO:0072756, GO:0072759, cellular response to boron-containing substance levels [GO:0080029], cellular response to toxic substance [GO:0097237], cellular response to peptide [GO:1901653], GO:1901699, cellular response to oxygen-containing compound [GO:1901701], cellular response to salt [GO:1902075], cellular response to N-phenylthiourea [GO:1902611], cellular response to fluoride [GO:1902618], cellular response to alkane [GO:1902779], GO:1903166, cellular response to cyanide [GO:1903928], cellular response to Aroclor 1254 [GO:1904011], GO:1904017, GO:1904148, GO:1904611, GO:1904613, GO:1904615, cellular response to dimethyl sulfoxide [GO:1904620], cellular response to hydrogen sulfide [GO:1904881], cellular response to phenylpropanoid [GO:1905546]